negative regulation of pancreatic stellate cell proliferation [GO:2000230] (biological process) Definition: Any process that stops, prevents, or reduces the frequency, rate or extent of pancreatic stellate cell proliferation. Relationships: is a type of negative regulation of fibroblast proliferation [GO:0048147]; is a type of regulation of pancreatic stellate cell proliferation [GO:2000229]; negatively regulates pancreatic stellate cell proliferation [GO:0072343] Sources: GOC:mah